{
  "term_id": "GO:0003700",
  "gene_name": "Zinc finger protein Eos",
  "gene": "UniProtKB:Q9H2S9",
  "term_label": "DNA-binding transcription factor activity",
  "gene_symbol": "IKZF4"
}